{
  "term_label": "structural constituent of ribosome",
  "gene_name": "Large ribosomal subunit protein uL10",
  "gene_symbol": "RPLP0",
  "term_id": "GO:0003735",
  "gene": "UniProtKB:P05388"
}